{
  "term_label": "endoplasmic reticulum",
  "term_id": "GO:0005783",
  "gene_name": "AN1-type zinc finger protein 2A",
  "gene_symbol": "ZFAND2A",
  "gene": "UniProtKB:Q8N6M9"
}